toluene-sulfonate methyl-monooxygenase activity [GO:0018652] (molecular function) Sources: RHEA:51024 Also known as: toluene-sulphonate methyl-monooxygenase activity Definition: Catalysis of the reaction: toluene-4-sulfonate + NADH + O2 = NAD+ + OH- + 4-sulfobenzyl alcohol. Relationships: is a type of oxidoreductase activity, acting on paired donors, with incorporation or reduction of molecular oxygen, NAD(P)H as one donor, and incorporation of one atom of oxygen [GO:0016709]